positive regulation of immune effector process [GO:0002699] (biological process) Sources: GOC:add Definition: Any process that activates or increases the frequency, rate, or extent of an immune effector process. Relationships: is_a positive regulation of immune system process [GO:0002684]; is a type of regulation of immune effector process [GO:0002697]; RO_0002213 immune effector process [GO:0002252] Subtypes: positive regulation of granuloma formation [GO:0002633], GO:0002702, positive regulation of leukocyte mediated immunity [GO:0002705], positive regulation of natural killer cell proliferation involved in immune response [GO:0032822], GO:0032828, positive regulation of CD4-positive, CD25-positive, alpha-beta regulatory T cell differentiation involved in immune response [GO:0032834], regulation of mast cell activation involved in immune response [GO:0033006], GO:0043302, GO:0043382, positive regulation of T-helper cell differentiation [GO:0045624], GO:0045917, positive regulation of respiratory burst involved in inflammatory response [GO:0060265], positive regulation of immune complex clearance by monocytes and macrophages [GO:0090265], positive regulation of plasma cell differentiation [GO:1900100], positive regulation of MDA-5 signaling pathway [GO:1900245], positive regulation of opsonization [GO:1903028], positive regulation of Fc-gamma receptor signaling pathway involved in phagocytosis [GO:1905451], positive regulation of T cell activation via T cell receptor contact with antigen bound to MHC molecule on antigen presenting cell [GO:2001190], GO:2001193 Also known as: up regulation of immune effector process, up-regulation of immune effector process, upregulation of immune effector process, activation of immune effector process, stimulation of immune effector process